{
  "term_id": "GO:0016712",
  "gene_symbol": "CYP2C19",
  "gene": "UniProtKB:P33261",
  "term_label": "oxidoreductase activity, acting on paired donors, with incorporation or reduction of molecular oxygen, reduced flavin or flavoprotein as one donor, and incorporation of one atom of oxygen",
  "gene_name": "Cytochrome P450 2C19"
}